signal clustering [GO:1990256] (biological process) Definition: Grouping of multiple copies of a signal at a cellular location. May promote receptor clustering and alter the signal transduction response. Also known as: ligand clustering Relationships: is a type of GO:0009966 References: PMID:12011072, PMID:15603739 Sources: GOC:als